{
  "gene_symbol": "GPATCH8",
  "gene_name": "G patch domain-containing protein 8",
  "term_label": "Unknown molecular function",
  "gene": "UniProtKB:Q9UKJ3",
  "term_id": "UNKNOWN:0001"
}